{
  "gene_name": "Zinc finger protein 844",
  "term_label": "nucleus",
  "gene": "UniProtKB:Q08AG5",
  "term_id": "GO:0005634",
  "gene_symbol": "ZNF844"
}